{
  "gene": "UniProtKB:P03973",
  "term_id": "GO:0045087",
  "gene_symbol": "SLPI",
  "term_label": "innate immune response",
  "gene_name": "Antileukoproteinase"
}